{
  "gene_name": "BRISC complex subunit Abraxas 2",
  "gene": "UniProtKB:Q15018",
  "gene_symbol": "ABRAXAS2",
  "term_id": "GO:0008017",
  "term_label": "microtubule binding"
}